cellular response to 4-nitroquinoline N-oxide [GO:0072725] (biological process) Relationships: is a type of response to 4-nitroquinoline N-oxide [GO:0072724]; is a type of cellular response to nitrogen compound [GO:1901699]; is a type of cellular response to oxygen-containing compound [GO:1901701] Sources: GOC:mah Definition: Any process that results in a change in state or activity of a cell (in terms of movement, secretion, enzyme production, gene expression, etc.) as a result of a 4-nitroquinoline N-oxide stimulus.